aldosterone catabolic process [GO:0032343] (biological process) Definition: The chemical reactions and pathways resulting in the breakdown of aldosterone, a corticosteroid hormone that is produced by the zona glomerulosa of the adrenal cortex and regulates salt (sodium and potassium) and water balance. References: PMID:16527843 Relationships: is_a GO:0006712; is a type of C21-steroid hormone catabolic process [GO:0008208]; is a type of aldosterone metabolic process [GO:0032341]; is a type of primary alcohol catabolic process [GO:0034310]; is a type of GO:0042182; is a type of GO:0046185; is a type of olefinic compound catabolic process [GO:0120256]